{
  "gene_name": "StAR-related lipid transfer protein 3",
  "gene": "UniProtKB:Q14849",
  "gene_symbol": "STARD3",
  "term_label": "endoplasmic reticulum membrane",
  "term_id": "GO:0005789"
}